{
  "gene": "UniProtKB:Q3MIR4",
  "term_id": "GO:0005794",
  "term_label": "Golgi apparatus",
  "gene_name": "Cell cycle control protein 50B",
  "gene_symbol": "TMEM30B"
}